{
  "gene_symbol": "PHF1",
  "term_label": "DNA binding",
  "gene_name": "PHD finger protein 1",
  "gene": "UniProtKB:O43189",
  "term_id": "GO:0003677"
}